maintenance of blood-brain barrier [GO:0035633] (biological process) Also known as: maintenance of BBB, maintenance of blood/brain barrier Definition: Maintaining the structure and function of the blood-brain barrier, thus ensuring specific regulated transport of substances (e.g. macromolecules, small molecules, ions) into the brain, and out of the brain into the blood circulation. References: PMID:20080302, PMID:30280653 Sources: GOC:aruk, GOC:bc, GOC:bf, GOC:sl Relationships: is a type of tissue homeostasis [GO:0001894] Note: Homeostasis and maintenance processes are regulatory processes, therefore, regulation child terms, such as: regulation of maintenance of blood-brain barrier, should not exist for these terms. 
Instead, for capturing regulation at the blood-brain barrier, consider using the part_of child term: regulation of blood-brain barrier permeability.